{
  "gene": "UniProtKB:Q8IXE1",
  "term_id": "GO:0005886",
  "gene_name": "Olfactory receptor 4N5",
  "gene_symbol": "OR4N5",
  "term_label": "plasma membrane"
}